negative regulation of endoplasmic reticulum stress-induced eIF2 alpha phosphorylation [GO:1903912] (biological process) Also known as: down regulation of eiF2alpha phosphorylation in response to ER stress, down regulation of eiF2alpha phosphorylation in response to endoplasmic reticulum stress, down regulation of regulation of translation initiation by eiF2alpha phosphorylation in response to endoplasmic reticulum stress, down-regulation of eiF2alpha phosphorylation in response to ER stress, down-regulation of eiF2alpha phosphorylation in response to endoplasmic reticulum stress, down-regulation of regulation of translation initiation by eiF2alpha phosphorylation in response to endoplasmic reticulum stress, downregulation of eiF2alpha phosphorylation in response to ER stress, downregulation of eiF2alpha phosphorylation in response to endoplasmic reticulum stress, downregulation of regulation of translation initiation by eiF2alpha phosphorylation in response to endoplasmic reticulum stress, negative regulation of ER stress-induced eIF2 alpha phosphorylation, negative regulation of eiF2alpha phosphorylation in response to ER stress, negative regulation of eiF2alpha phosphorylation in response to endoplasmic reticulum stress, negative regulation of regulation of translation initiation by eiF2alpha phosphorylation in response to endoplasmic reticulum stress, inhibition of eiF2alpha phosphorylation in response to ER stress, inhibition of eiF2alpha phosphorylation in response to endoplasmic reticulum stress, inhibition of regulation of translation initiation by eiF2alpha phosphorylation in response to endoplasmic reticulum stress References: PMID:16835242 Sources: GOC:PARL, GOC:TermGenie, GOC:bf, GO_REF:0000058 Relationships: is a type of negative regulation of protein phosphorylation [GO:0001933]; is a type of GO:0006446; negatively regulates GO:0036492 Definition: Any process that stops, prevents or reduces the frequency, rate or extent of endoplasmic reticulum stress-induced eiF2alpha phosphorylation.